{
  "gene_symbol": "NR1I2",
  "term_id": "GO:0000978",
  "gene": "UniProtKB:O75469",
  "term_label": "RNA polymerase II cis-regulatory region sequence-specific DNA binding",
  "gene_name": "Nuclear receptor subfamily 1 group I member 2"
}